{
  "gene_symbol": "COX17",
  "term_label": "mitochondrial respiratory chain complex IV assembly",
  "term_id": "GO:0033617",
  "gene_name": "Cytochrome c oxidase copper chaperone",
  "gene": "UniProtKB:Q14061"
}